regulation of ammonia assimilation cycle [GO:2001248] (BP) Definition: Any process that modulates the frequency, rate or extent of ammonia assimilation cycle. Sources: GOC:BHF Relationships: is a type of GO:0006808; is a type of regulation of glutamate metabolic process [GO:2000211]; regulates ammonia assimilation cycle [GO:0019676] Also known as: regulation of glutamate metabolic process via glutamine and ammonia, regulation of glutamate metabolism via glutamine and ammonia Subtypes: GO:2001249, positive regulation of ammonia assimilation cycle [GO:2001250]